{
  "gene_symbol": "LMAN1",
  "gene_name": "Protein ERGIC-53",
  "term_label": "endoplasmic reticulum to Golgi vesicle-mediated transport",
  "term_id": "GO:0006888",
  "gene": "UniProtKB:P49257"
}